{
  "term_id": "GO:0000462",
  "gene_symbol": "NGDN",
  "term_label": "maturation of SSU-rRNA from tricistronic rRNA transcript (SSU-rRNA, 5.8S rRNA, LSU-rRNA)",
  "gene_name": "Neuroguidin",
  "gene": "UniProtKB:Q8NEJ9"
}